{
  "term_id": "GO:0004666",
  "term_label": "prostaglandin-endoperoxide synthase activity",
  "gene_name": "Prostaglandin G_H synthase 1",
  "gene": "UniProtKB:P23219",
  "gene_symbol": "PTGS1"
}